rhombomere structural organization [GO:0021595] (BP) Subtypes: rhombomere 1 structural organization [GO:0021653], rhombomere 2 structural organization [GO:0021656], rhombomere 3 structural organization [GO:0021659], rhombomere 4 structural organization [GO:0021662], GO:0021665, rhombomere 6 structural organization [GO:0021668], rhombomere 7 structural organization [GO:0021672], GO:0021676 Sources: GOC:cls, GOC:dgh, GOC:dph, GOC:jid, GO_REF:0000021 Relationships: is a type of anatomical structure arrangement [GO:0048532]; is part of GO:0021593 Also known as: rhombomere structural organisation Definition: The process that contributes to the act of creating the structural organization of the rhombomere structure. Rhombomeres are transverse segments of the developing rhombencephalon. Rhombomeres are lineage restricted, express different genes from one another, and adopt different developmental fates.